{
  "term_label": "nucleus",
  "term_id": "GO:0005634",
  "gene_symbol": "ZNF121",
  "gene": "UniProtKB:P58317",
  "gene_name": "Zinc finger protein 121"
}